cytidine transport [GO:0015861] (biological process) Sources: GOC:go_curators Relationships: is a type of GO:0015864 Definition: The directed movement of cytidine, cytosine riboside, into, out of or within a cell, or between cells, by means of some agent such as a transporter or pore.